{
  "term_label": "extracellular matrix organization",
  "term_id": "GO:0030198",
  "gene_symbol": "COL9A1",
  "gene": "UniProtKB:P20849",
  "gene_name": "Collagen alpha-1(IX) chain"
}